beta-carotene catabolic process [GO:1901811] (biological process) Also known as: beta-carotene breakdown, beta-carotene catabolism, beta-carotene degradation Relationships: is_a GO:0016118; is a type of carotene catabolic process [GO:0016121]; is a type of beta-carotene metabolic process [GO:1901810] Definition: The chemical reactions and pathways resulting in the breakdown of beta-carotene. References: PMID:11387982 Sources: GOC:TermGenie, GOC:yaf, MetaCyc:PWY-5943, UniPathway:UPA00802